{
  "gene": "UniProtKB:O60381",
  "term_id": "GO:0000978",
  "gene_name": "HMG box-containing protein 1",
  "gene_symbol": "HBP1",
  "term_label": "RNA polymerase II cis-regulatory region sequence-specific DNA binding"
}